{
  "gene": "UniProtKB:Q9Y3R5",
  "gene_symbol": "DOP1B",
  "gene_name": "Protein dopey-2",
  "term_label": "trans-Golgi network",
  "term_id": "GO:0005802"
}